{
  "term_id": "GO:0031667",
  "term_label": "response to nutrient levels",
  "gene": "UniProtKB:Q14406",
  "gene_name": "Chorionic somatomammotropin hormone-like 1",
  "gene_symbol": "CSHL1"
}